{
  "term_label": "regulation of translation at presynapse, modulating synaptic transmission",
  "gene_symbol": "FXR2",
  "gene": "UniProtKB:P51116",
  "term_id": "GO:0099577",
  "gene_name": "RNA-binding protein FXR2"
}